{
  "gene_name": "Membrane-associated progesterone receptor component 2",
  "gene_symbol": "PGRMC2",
  "gene": "UniProtKB:O15173",
  "term_label": "endoplasmic reticulum",
  "term_id": "GO:0005783"
}